{
  "gene_symbol": "LINC02906",
  "term_label": "Unknown biological process",
  "gene": "UniProtKB:E5RJ46",
  "term_id": "UNKNOWN:0002",
  "gene_name": "Putative uncharacterized protein LINC02906"
}